{
  "gene_symbol": "MUC6",
  "term_id": "GO:0031012",
  "gene_name": "Mucin-6",
  "gene": "UniProtKB:Q6W4X9",
  "term_label": "extracellular matrix"
}